{
  "term_id": "GO:0050870",
  "gene": "UniProtKB:P28067",
  "gene_name": "HLA class II histocompatibility antigen, DM alpha chain",
  "gene_symbol": "HLA-DMA",
  "term_label": "positive regulation of T cell activation"
}